{
  "gene_symbol": "SERPINC1",
  "gene": "UniProtKB:P01008",
  "term_label": "serine-type endopeptidase inhibitor activity",
  "term_id": "GO:0004867",
  "gene_name": "Antithrombin-III"
}